tagatose-bisphosphate aldolase activity [GO:0009025] (molecular function) Relationships: is a type of aldehyde-lyase activity [GO:0016832] Sources: EC:4.1.2.40, RHEA:22948 Definition: Catalysis of the reaction: D-tagatose 1,6-diphosphate = D-glyceraldehyde 3-phosphate + glycerone phosphate. Also known as: D-tagatose-1,6-bisphosphate triosephosphate lyase activity, tagatose-1,6-bisphosphate aldolase 1, AgaY, AgaZ, D-tagatose-1,6-bisphosphate D-glyceraldehyde 3-phosphate-lyase (glycerone-phosphate-forming), D-tagatose-1,6-bisphosphate aldolase activity, KbaY, tagatose 1,6-diphosphate aldolase activity